{
  "term_label": "termination of RNA polymerase II transcription",
  "gene": "UniProtKB:Q9UPN6",
  "term_id": "GO:0006369",
  "gene_symbol": "SCAF8",
  "gene_name": "SR-related and CTD-associated factor 8"
}